{
  "gene_symbol": "SLC9A5",
  "gene": "UniProtKB:Q14940",
  "term_id": "GO:0015386",
  "term_label": "potassium:proton antiporter activity",
  "gene_name": "Sodium_hydrogen exchanger 5"
}